{
  "term_label": "positive regulation of synaptic transmission, glutamatergic",
  "gene_symbol": "CACNG7",
  "gene": "UniProtKB:P62955",
  "gene_name": "Voltage-dependent calcium channel gamma-7 subunit",
  "term_id": "GO:0051968"
}